{
  "term_label": "nucleus",
  "term_id": "GO:0005634",
  "gene": "UniProtKB:O94842",
  "gene_symbol": "TOX4",
  "gene_name": "TOX high mobility group box family member 4"
}